myelin sheath [GO:0043209] (cellular component) Definition: An electrically insulating fatty layer that surrounds the axons of many neurons. It is an outgrowth of glial cells: Schwann cells supply the myelin for peripheral neurons while oligodendrocytes supply it to those of the central nervous system. Also known as: Schwann cell myelin sheath, astrocyte sheath, oligodendrocyte myelin sheath Relationships: is a type of cellular anatomical structure [GO:0110165] Sources: GOC:cjm, GOC:jl, NIF_Subcellular:sao593830697, Wikipedia:Myelin